high-affinity glutamine transmembrane transporter activity [GO:0015330] (molecular function) Definition: Enables the transfer of glutamine from one side of a membrane to the other. In high-affinity transport the transporter is able to bind the solute even if it is only present at very low concentrations. Also known as: high affinity glutamine transmembrane transporter activity, high affinity glutamine permease activity Relationships: is a type of GO:0005287; is a type of GO:0015186 Sources: GOC:mtg_transport